myosin tail binding [GO:0032029] (molecular function) Subtypes: myosin I tail binding [GO:0032032], myosin II tail binding [GO:0032035], myosin XI tail binding [GO:0080115] Sources: GOC:mah Relationships: is a type of GO:0032036 Definition: Binding to the tail region of a myosin heavy chain.